{
  "gene_name": "Submaxillary gland androgen-regulated protein 3A",
  "term_id": "GO:0004866",
  "gene_symbol": "SMR3A",
  "gene": "UniProtKB:Q99954",
  "term_label": "endopeptidase inhibitor activity"
}